integrin alpha6-beta1 complex [GO:0034675] (cellular component) References: PMID:12297042 Definition: An integrin complex that comprises one alpha6 subunit and one beta1 subunit. Also known as: VLA-6 complex, alpha6-beta1 integrin complex, ITGA6-ITGB1 complex Relationships: is a type of GO:0008305